{
  "term_label": "Unknown molecular function",
  "term_id": "UNKNOWN:0001",
  "gene": "UniProtKB:A6NEF3",
  "gene_symbol": "GOLGA6L4",
  "gene_name": "Golgin subfamily A member 6-like protein 4"
}